hindbrain morphogenesis [GO:0021575] (biological process) Relationships: is a type of GO:0009653; is part of hindbrain development [GO:0030902] Sources: GOC:cls, GOC:dgh, GOC:dph, GOC:jid, GO_REF:0000021 Definition: The process in which the anatomical structure of the hindbrain is generated and organized. The hindbrain is the region consisting of the medulla, pons and cerebellum. Areas of the hindbrain control motor and autonomic functions. Also known as: rhombencephalon morphogenesis